mast cell apoptotic process [GO:0033024] (biological process) Also known as: apoptosis of mast cells, mast cell apoptosis References: PMID:11292031, PMID:12360215, PMID:16605130 Sources: CL:0000097, GOC:add, GOC:mtg_apoptosis Definition: Any apoptotic process in a mast cell, a cell that is found in almost all tissues containing numerous basophilic granules and capable of releasing large amounts of histamine and heparin upon activation. Regulation: regulated by regulation of mast cell apoptotic process [GO:0033025]; negatively regulated by negative regulation of mast cell apoptotic process [GO:0033026]; positively regulated by positive regulation of mast cell apoptotic process [GO:0033027] Relationships: is a type of myeloid cell apoptotic process [GO:0033028]; is a type of leukocyte apoptotic process [GO:0071887]; is part of mast cell homeostasis [GO:0033023]